multiple spine synapse organization [GO:0150089] (biological process) Definition: A process that is carried out at the cellular level which results in the assembly, arrangement of constituent parts, or disassembly of a synapse between a multiple synapse bouton and one or more dendritic spines. References: PMID:10586883, PMID:11248111, PMID:11466428, PMID:18501438, PMID:22028887, PMID:29774619, PMID:7482800, PMID:8366344 Sources: GOC:aruk, GOC:bc Also known as: multi-synapse organisation, multi-synapse organization, multi-synaptic organisation, multi-synaptic organization, multisynapse organisation, multisynapse organization, multisynaptic organisation, multisynaptic organization, multiple spine synapse organisation Relationships: is a type of synapse organization [GO:0050808] Subtypes: GO:0150090, multiple spine synapse organization, multiple dendrites [GO:0150091]